{
  "gene_symbol": "EIF4E2",
  "gene": "UniProtKB:O60573",
  "term_id": "GO:0003743",
  "gene_name": "Eukaryotic translation initiation factor 4E type 2",
  "term_label": "translation initiation factor activity"
}